{
  "gene_name": "Transcription factor 12",
  "gene_symbol": "TCF12",
  "term_id": "GO:0005667",
  "gene": "UniProtKB:Q99081",
  "term_label": "transcription regulator complex"
}